{
  "term_id": "GO:0000978",
  "gene": "UniProtKB:O15156",
  "gene_symbol": "ZBTB7B",
  "gene_name": "Zinc finger and BTB domain-containing protein 7B",
  "term_label": "RNA polymerase II cis-regulatory region sequence-specific DNA binding"
}